export from the mitochondrion [GO:0170037] (biological process) Sources: GOC:ew Subtypes: GO:0019090 Definition: The directed movement of substances from the mitochondrion to the cytosol. Relationships: is a type of mitochondrial transmembrane transport [GO:1990542]